dendrite morphogenesis [GO:0048813] (biological process) Subtypes: GO:0140059, GO:0150019, apical dendrite morphogenesis [GO:0150021] Regulation: regulated by regulation of dendrite morphogenesis [GO:0048814]; negatively regulated by GO:0050774; positively regulated by positive regulation of dendrite morphogenesis [GO:0050775] References: PMID:22683681 Sources: GOC:aruk, GOC:bc, GOC:jl, ISBN:0198506732 Relationships: is a type of neuron projection morphogenesis [GO:0048812]; is part of dendrite development [GO:0016358]; is part of cell morphogenesis involved in neuron differentiation [GO:0048667] Definition: The process in which the anatomical structures of a dendrite are generated and organized.